{
  "gene": "UniProtKB:P09017",
  "gene_name": "Homeobox protein Hox-C4",
  "gene_symbol": "HOXC4",
  "term_label": "DNA-binding transcription factor activity, RNA polymerase II-specific",
  "term_id": "GO:0000981"
}